arsenite transmembrane transporter activity [GO:0015105] (molecular function) Subtypes: GO:0008490 Definition: Enables the transfer of arsenite from one side of a membrane to the other. Sources: GOC:ai Relationships: is a type of transmembrane transporter activity [GO:0022857]; is part of arsenite transport [GO:0015700]